negative regulation of terminal cell fate specification, open tracheal system [GO:0035155] (biological process) Relationships: is_a negative regulation of cell fate specification [GO:0009996]; is a type of negative regulation of multicellular organismal process [GO:0051241]; RO_0002212 terminal cell fate specification, open tracheal system [GO:0035154] Also known as: down regulation of terminal cell fate specification, down-regulation of terminal cell fate specification, downregulation of terminal cell fate specification, negative regulation of terminal cell fate specification, inhibition of terminal cell fate specification References: PMID:10684581 Sources: GOC:mtg_sensu Definition: Any process that restricts, stops or prevents a cell from adopting a terminal cell fate in an open tracheal system. Once the terminal and fusion fates have been correctly induced, inhibitory feedback loops prevent the remaining branch cells from assuming similar fates.